{
  "gene": "UniProtKB:Q9NVV5",
  "gene_name": "Androgen-induced gene 1 protein",
  "term_id": "UNKNOWN:0002",
  "gene_symbol": "AIG1",
  "term_label": "Unknown biological process"
}